D-inositol-3-phosphate glycosyltransferase activity [GO:0102710] (molecular function) Sources: GOC:pz, RHEA:26188 Relationships: is a type of hexosyltransferase activity [GO:0016758] Definition: Catalysis of the reaction: UDP-N-acetyl-alpha-D-glucosamine + 1D-myo-inositol 3-phosphate = 1D-myo-inositol 2-acetamido-2-deoxy-alpha-D-glucopyranoside 3-phosphate + UDP + H+.